{
  "gene": "UniProtKB:O75943",
  "gene_symbol": "RAD17",
  "term_label": "chromatin",
  "term_id": "GO:0000785",
  "gene_name": "Cell cycle checkpoint protein RAD17"
}